{
  "gene": "UniProtKB:Q9P2E7",
  "term_label": "plasma membrane",
  "term_id": "GO:0005886",
  "gene_name": "Protocadherin-10",
  "gene_symbol": "PCDH10"
}